{
  "gene": "UniProtKB:P01889",
  "gene_name": "HLA class I histocompatibility antigen, B alpha chain",
  "term_id": "GO:0005102",
  "gene_symbol": "HLA-B",
  "term_label": "signaling receptor binding"
}